{
  "term_label": "taurine transmembrane transport",
  "gene": "UniProtKB:P31641",
  "gene_name": "Sodium- and chloride-dependent taurine transporter",
  "gene_symbol": "SLC6A6",
  "term_id": "GO:0015734"
}